abieta-7,13-diene hydroxylase activity [GO:0036189] (molecular function) Definition: Catalysis of the reaction: abieta-7,13-diene + NADPH + H+ + O2 = abieta-7,13-dien-18-ol + NADP+ + H2O. Also known as: abietadiene hydroxylase Relationships: is_a oxidoreductase activity, acting on paired donors, with incorporation or reduction of molecular oxygen, NAD(P)H as one donor, and incorporation of one atom of oxygen [GO:0016709] Sources: EC:1.14.14.144